left caudal basal body [GO:1902677] (cellular component) Note: Note that we deem cilium and microtubule-based flagellum to be equivalent. Also note that, due to the asymmetric nature of the Giardia trophozoite, this term is defined spatially as the trophozoite is viewed from the dorsal side, with the two nuclei dorsal to the ventral disc, and the ventral disc toward the anterior. Relationships: is a type of ciliary basal body [GO:0036064]; is part of left caudal flagellum [GO:0097560] Also known as: cilial basal body of left caudal cilium, cilial basal body of left caudal flagellum, ciliary basal body of left caudal cilium, ciliary basal body of left caudal flagellum, cilium basal body of left caudal cilium, cilium basal body of left caudal flagellum, left caudal flagellum ciliary basal body, microtubule basal body of left caudal cilium, microtubule basal body of left caudal flagellum References: PMID:16607022, PMID:5961344 Sources: GOC:TermGenie, GOC:giardia, GO_REF:0000064, ISBN:9780124260207 Definition: Any ciliary basal body that is part of a left caudal flagellum found in Giardia species (trophozoite stage).